polycistronic mRNA processing [GO:0031426] (biological process) Definition: The conversion of a primary mRNA transcript containing more than one complete protein-coding region into individual mature mRNA molecules. Sources: GOC:mah Relationships: is a type of GO:0006397